{
  "gene": "UniProtKB:Q6PP77",
  "gene_name": "XK-related protein 2",
  "gene_symbol": "XKRX",
  "term_id": "UNKNOWN:0003",
  "term_label": "Unknown cellular component"
}